{
  "gene_symbol": "MORN5",
  "term_id": "UNKNOWN:0002",
  "gene": "UniProtKB:Q5VZ52",
  "gene_name": "MORN repeat-containing protein 5",
  "term_label": "Unknown biological process"
}